{
  "gene_name": "Putative ankyrin repeat domain-containing protein 20A2",
  "gene_symbol": "ANKRD20A2P",
  "gene": "UniProtKB:Q5SQ80",
  "term_label": "Unknown biological process",
  "term_id": "UNKNOWN:0002"
}